{
  "term_label": "cholesterol binding",
  "gene": "UniProtKB:Q9UHC9",
  "term_id": "GO:0015485",
  "gene_name": "NPC1-like intracellular cholesterol transporter 1",
  "gene_symbol": "NPC1L1"
}